{
  "term_label": "lipid metabolic process",
  "gene_symbol": "LIPK",
  "gene": "UniProtKB:Q5VXJ0",
  "term_id": "GO:0006629",
  "gene_name": "Lipase member K"
}